ganglioside catabolic process [GO:0006689] (biological process) Sources: ISBN:0198547684 Definition: The chemical reactions and pathways resulting in the breakdown of ganglioside, a ceramide oligosaccharide carrying, in addition to other sugar residues, one or more sialic residues. Also known as: ganglioside breakdown, ganglioside catabolism, ganglioside degradation Relationships: is a type of ganglioside metabolic process [GO:0001573]; is a type of glycosphingolipid catabolic process [GO:0046479]; is a type of ceramide catabolic process [GO:0046514]